isoleucine metabolic process [GO:0006549] (biological process) Sources: GOC:ai Relationships: is a type of branched-chain amino acid metabolic process [GO:0009081]; is a type of GO:1901605 Definition: The chemical reactions and pathways involving isoleucine, (2R*,3R*)-2-amino-3-methylpentanoic acid. Subtypes: L-isoleucine catabolic process [GO:0006550], isoleucine biosynthetic process [GO:0009097] Also known as: isoleucine metabolism